{
  "gene_symbol": "FOXG1",
  "gene_name": "Forkhead box protein G1",
  "term_id": "GO:0005634",
  "gene": "UniProtKB:P55316",
  "term_label": "nucleus"
}